{
  "gene_symbol": "PFKM",
  "gene_name": "ATP-dependent 6-phosphofructokinase, muscle type",
  "term_label": "canonical glycolysis",
  "term_id": "GO:0061621",
  "gene": "UniProtKB:P08237"
}